{
  "term_id": "UNKNOWN:0001",
  "term_label": "Unknown molecular function",
  "gene": "UniProtKB:Q9HB20",
  "gene_name": "Pleckstrin homology domain-containing family A member 3",
  "gene_symbol": "PLEKHA3"
}